base conversion or substitution editing [GO:0016553] (biological process) Definition: Any base modification or substitution events that result in alterations in the coding potential or structural properties of RNAs as a result of changes in the base-pairing properties of the modified ribonucleoside(s). References: PMID:11092837 Also known as: base conversion/substitution editing Relationships: is a type of GO:0009451 Subtypes: GO:0006382, cytidine to uridine editing [GO:0016554], uridine to cytidine editing [GO:0016555]